{
  "term_label": "endoplasmic reticulum membrane",
  "gene": "UniProtKB:Q96CP6",
  "gene_symbol": "GRAMD1A",
  "gene_name": "Protein Aster-A",
  "term_id": "GO:0005789"
}